2-hydroxymuconate-semialdehyde hydrolase activity [GO:0018775] (molecular function) Also known as: 2-hydroxymuconate-semialdehyde formylhydrolase activity, 2-hydroxymuconic semialdehyde hydrolase activity, HMSH, HOD hydrolase activity Relationships: is a type of hydrolase activity, acting on acid carbon-carbon bonds, in ketonic substances [GO:0016823] Sources: RHEA:14549 Definition: Catalysis of the reaction: (2Z,4E)-2-hydroxy-6-oxohexa-2,4-dienoate + H2O = 2-oxopent-4-enoate + formate + H+.